zinc efflux antiporter activity [GO:0015341] (molecular function) Definition: Enables the transfer of a zinc ion or zinc ions from the inside of the cell to the outside of the cell across a membrane according to the reaction H+(out) + Zn2+(in) = H+(in) + Zn2+(out). The activity is driven by proton motive force. References: PMID:35226479 Sources: GOC:mtg_transport, ISBN:0815340729, TC:2.A.4.1.4, TC:2.A.4.2.3 Also known as: zinc efflux permease activity Relationships: is a type of GO:0140826